asparagine-oxo-acid transaminase activity [GO:0047297] (molecular function) Definition: Catalysis of the reaction: a 2-oxo acid + L-asparagine = an amino acid + 2-oxosuccinamate. Also known as: asparagine-oxo-acid aminotransferase activity, L-asparagine:2-oxo-acid aminotransferase activity, asparagine--oxo-acid aminotransferase activity, asparagine-keto acid aminotransferase activity Relationships: is a type of transaminase activity [GO:0008483] Sources: RHEA:19813